{
  "gene_symbol": "SLC25A13",
  "term_label": "L-aspartate transmembrane transporter activity",
  "gene_name": "Electrogenic aspartate_glutamate antiporter SLC25A13, mitochondrial",
  "gene": "UniProtKB:Q9UJS0",
  "term_id": "GO:0015183"
}